nucleotidyltransferase activity [GO:0016779] (MF) Definition: Catalysis of the transfer of a nucleotidyl group from one compound (donor) to another (acceptor). Relationships: is_a transferase activity, transferring phosphorus-containing groups [GO:0016772] Subtypes: polyribonucleotide nucleotidyltransferase activity [GO:0004654], GO:0008879, tRNA nucleotidyltransferase activity [GO:0009022], lipoate-protein ligase activity [GO:0016979], GO:0017125, DNA polymerase activity [GO:0034061], aminoglycoside nucleotidyltransferase activity [GO:0034068], nucleoside-triphosphate-hexose-1-phosphate nucleotidyltransferase activity [GO:0047339], galactose-1-phosphate thymidylyltransferase activity [GO:0047342], aldose-1-phosphate nucleotidyltransferase activity [GO:0047347], [glutamine synthetase]-adenylyl-L-tyrosine phosphorylase activity [GO:0047388], holo-citrate lyase synthase activity [GO:0050519], diguanylate cyclase activity [GO:0052621], L-threonylcarbamoyladenylate synthase [GO:0061710], adenylyltransferase activity [GO:0070566], cytidylyltransferase activity [GO:0070567], guanylyltransferase activity [GO:0070568], uridylyltransferase activity [GO:0070569], GO:0097747, GO:0098680, diadenylate cyclase activity [GO:0106408], cyclic-di-AMP phosphodiesterase activity [GO:0106409], cyclic GMP-AMP synthase activity [GO:0140699], guanylylpyridinol adenylase activity [GO:0160301] Sources: EC:2.7.7.-